{
  "gene_name": "P2Y purinoceptor 1",
  "term_id": "GO:0005886",
  "gene": "UniProtKB:P47900",
  "term_label": "plasma membrane",
  "gene_symbol": "P2RY1"
}